{
  "term_label": "chloride channel complex",
  "term_id": "GO:0034707",
  "gene_name": "H(+)_Cl(-) exchange transporter 7",
  "gene_symbol": "CLCN7",
  "gene": "UniProtKB:P51798"
}